{
  "term_id": "UNKNOWN:0002",
  "term_label": "Unknown biological process",
  "gene_name": "Uncharacterized protein C12orf42",
  "gene": "UniProtKB:Q96LP6",
  "gene_symbol": "C12orf42"
}